negative regulation of dermatome development [GO:0061185] (BP) Sources: GOC:BHF, GOC:dph Relationships: is_a negative regulation of embryonic development [GO:0045992]; is a type of regulation of dermatome development [GO:0061183]; negatively regulates dermatome development [GO:0061054] Definition: Any process that decreases the rate, frequency, or extent of the progression of the dermatome over time, from its initial formation to the mature structure. The dermatome is the portion of a somite that will form skin.